signal recognition particle, chloroplast targeting [GO:0080085] (cellular component) Relationships: is a type of signal recognition particle [GO:0048500] References: PMID:17513500 Definition: A complex consisting of a protein and RNA component which binds the signal sequence of some proteins and facilitates their export to the chloroplast.